RNA decapping [GO:0110154] (biological process) Definition: Cleavage of the 5'-cap of an RNA. References: PMID:25533955, PMID:31101919 Sources: GOC:sp Relationships: is a type of RNA metabolic process [GO:0016070] Subtypes: GO:0110155, GO:0110156